{
  "term_id": "GO:0140374",
  "term_label": "antiviral innate immune response",
  "gene_symbol": "DHX58",
  "gene": "UniProtKB:Q96C10",
  "gene_name": "ATP-dependent RNA helicase DHX58"
}